{
  "term_id": "GO:0016034",
  "gene": "UniProtKB:O43708",
  "gene_name": "Maleylacetoacetate isomerase",
  "gene_symbol": "GSTZ1",
  "term_label": "maleylacetoacetate isomerase activity"
}